{
  "gene_name": "Homeobox protein NOBOX",
  "gene": "UniProtKB:O60393",
  "gene_symbol": "NOBOX",
  "term_id": "GO:0000978",
  "term_label": "RNA polymerase II cis-regulatory region sequence-specific DNA binding"
}